{
  "term_id": "GO:0036064",
  "gene": "UniProtKB:Q8TAM2",
  "term_label": "ciliary basal body",
  "gene_name": "Tetratricopeptide repeat protein 8",
  "gene_symbol": "TTC8"
}